{
  "gene_name": "Protein fem-1 homolog A",
  "term_id": "GO:0000151",
  "gene": "UniProtKB:Q9BSK4",
  "gene_symbol": "FEM1A",
  "term_label": "ubiquitin ligase complex"
}